{
  "gene": "UniProtKB:Q96LL4",
  "gene_symbol": "C8orf48",
  "term_id": "UNKNOWN:0003",
  "gene_name": "Uncharacterized protein C8orf48",
  "term_label": "Unknown cellular component"
}